{
  "gene": "UniProtKB:Q86V42",
  "term_label": "Unknown molecular function",
  "term_id": "UNKNOWN:0001",
  "gene_name": "Protein FAM124A",
  "gene_symbol": "FAM124A"
}